intermediate reticular formation development [GO:0021727] (biological process) Sources: GOC:cls, GOC:curators, GOC:dgh, GOC:dph, GOC:jid Relationships: is a type of GO:0048856; is part of medullary reticular formation development [GO:0021723] Definition: The process whose specific outcome is the progression of the intermediate reticular formation over time, from its formation to the mature structure. Also known as: intermediate reticular nucleus development